neural plate mediolateral regionalization [GO:0021998] (biological process) Definition: The process that regulates the coordinated growth and differentiation that establishes the non-random mediolateral spatial arrangement of the neural plate. Sources: GOC:cls, GOC:dgh, GOC:dph, GOC:jid, GO_REF:0000021 Also known as: neural plate mediolateral pattern formation Relationships: is a type of neural plate regionalization [GO:0060897]